peribacteroid fluid [GO:0043662] (cellular component) Relationships: is a type of cellular anatomical structure [GO:0110165]; is part of GO:0043660 Definition: The soluble material inside the peribacteroid membrane, but outside of the bacteroid, within a bacteroid-containing symbiosome. Sources: GOC:cc